{
  "term_id": "GO:0007507",
  "gene_symbol": "PRICKLE4",
  "gene": "UniProtKB:Q2TBC4",
  "term_label": "heart development",
  "gene_name": "Prickle-like protein 4"
}